{
  "gene_name": "Muscarinic acetylcholine receptor M5",
  "term_label": "adenylate cyclase-inhibiting G protein-coupled acetylcholine receptor signaling pathway",
  "gene_symbol": "CHRM5",
  "term_id": "GO:0007197",
  "gene": "UniProtKB:P08912"
}